{
  "term_id": "UNKNOWN:0003",
  "gene_name": "Apolipoprotein L6",
  "gene_symbol": "APOL6",
  "gene": "UniProtKB:Q9BWW8",
  "term_label": "Unknown cellular component"
}